{
  "term_id": "GO:0022625",
  "gene": "UniProtKB:P30050",
  "gene_name": "Large ribosomal subunit protein uL11",
  "term_label": "cytosolic large ribosomal subunit",
  "gene_symbol": "RPL12"
}